{
  "term_id": "UNKNOWN:0003",
  "gene": "UniProtKB:O95294",
  "gene_symbol": "RASAL1",
  "gene_name": "RasGAP-activating-like protein 1",
  "term_label": "Unknown cellular component"
}